{
  "gene": "UniProtKB:Q9H469",
  "gene_symbol": "FBXL15",
  "term_label": "Unknown molecular function",
  "gene_name": "F-box_LRR-repeat protein 15",
  "term_id": "UNKNOWN:0001"
}